{
  "gene": "UniProtKB:Q9UK85",
  "gene_name": "Dickkopf-like protein 1",
  "gene_symbol": "DKKL1",
  "term_id": "GO:0048019",
  "term_label": "receptor antagonist activity"
}